{
  "term_id": "GO:0005547",
  "gene_symbol": "ZFYVE1",
  "term_label": "phosphatidylinositol-3,4,5-trisphosphate binding",
  "gene": "UniProtKB:Q9HBF4",
  "gene_name": "Zinc finger FYVE domain-containing protein 1"
}